{
  "term_id": "GO:0005247",
  "gene_name": "Chloride channel protein ClC-Kb",
  "term_label": "voltage-gated chloride channel activity",
  "gene": "UniProtKB:P51801",
  "gene_symbol": "CLCNKB"
}